{
  "gene_symbol": "PPM1N",
  "term_label": "nucleus",
  "gene": "UniProtKB:Q8N819",
  "gene_name": "Probable protein phosphatase 1N",
  "term_id": "GO:0005634"
}